negative regulation of type B pancreatic cell proliferation [GO:1904691] (biological process) Also known as: down regulation of pancreatic B cell proliferation, down regulation of pancreatic beta cell proliferation, down regulation of type B pancreatic cell proliferation, down-regulation of pancreatic B cell proliferation, down-regulation of pancreatic beta cell proliferation, down-regulation of type B pancreatic cell proliferation, downregulation of pancreatic B cell proliferation, downregulation of pancreatic beta cell proliferation, downregulation of type B pancreatic cell proliferation, negative regulation of pancreatic B cell proliferation, negative regulation of pancreatic beta cell proliferation, inhibition of pancreatic B cell proliferation, inhibition of pancreatic beta cell proliferation, inhibition of type B pancreatic cell proliferation Definition: Any process that stops, prevents or reduces the frequency, rate or extent of type B pancreatic cell proliferation. References: PMID:24055447 Sources: GOC:TermGenie, GO_REF:0000058 Relationships: is_a negative regulation of epithelial cell proliferation [GO:0050680]; is a type of regulation of type B pancreatic cell proliferation [GO:0061469]; negatively regulates type B pancreatic cell proliferation [GO:0044342]